{
  "gene": "UniProtKB:P40238",
  "gene_symbol": "MPL",
  "term_label": "thrombopoietin receptor activity",
  "gene_name": "Thrombopoietin receptor",
  "term_id": "GO:0038164"
}